{
  "term_label": "cytosol",
  "term_id": "GO:0005829",
  "gene": "UniProtKB:P00973",
  "gene_name": "2'-5'-oligoadenylate synthase 1",
  "gene_symbol": "OAS1"
}